{
  "gene_name": "Phospholipid-transporting ATPase ABCA3",
  "term_label": "lipid transport",
  "term_id": "GO:0006869",
  "gene_symbol": "ABCA3",
  "gene": "UniProtKB:Q99758"
}